{
  "gene_name": "Spermatogenesis-associated serine-rich protein 1",
  "gene_symbol": "SPATS1",
  "term_id": "UNKNOWN:0003",
  "gene": "UniProtKB:Q496A3",
  "term_label": "Unknown cellular component"
}